{
  "gene_symbol": "MRPS21",
  "gene": "UniProtKB:P82921",
  "gene_name": "Small ribosomal subunit protein bS21m",
  "term_id": "UNKNOWN:0003",
  "term_label": "Unknown cellular component"
}